{
  "gene_symbol": "FAM76B",
  "term_label": "Unknown biological process",
  "gene_name": "Protein FAM76B",
  "term_id": "UNKNOWN:0002",
  "gene": "UniProtKB:Q5HYJ3"
}